{
  "gene_symbol": "ZNF48",
  "term_id": "GO:0006357",
  "gene": "UniProtKB:Q96MX3",
  "term_label": "regulation of transcription by RNA polymerase II",
  "gene_name": "Zinc finger protein 48"
}